tartronate-semialdehyde synthase activity [GO:0009028] (molecular function) Also known as: glyoxalate carboligase activity, glyoxylate carbo-ligase activity, glyoxylate carboligase activity, glyoxylate carboxy-lyase (dimerizing), glyoxylate carboxy-lyase (dimerizing; tartronate-semialdehyde-forming), glyoxylic carbo-ligase activity, hydroxymalonic semialdehyde carboxylase activity, tartronate semialdehyde carboxylase activity, tartronic semialdehyde carboxylase activity Definition: Catalysis of the reaction: 2 glyoxylate + H+ = 2-hydroxy-3-oxopropanoate + CO2. Relationships: is a type of carboxy-lyase activity [GO:0016831] Sources: EC:4.1.1.47, RHEA:10136